{
  "term_label": "integrator complex",
  "gene": "UniProtKB:Q96HW7",
  "gene_name": "Integrator complex subunit 4",
  "gene_symbol": "INTS4",
  "term_id": "GO:0032039"
}